{
  "gene": "UniProtKB:Q9NRM2",
  "gene_name": "Zinc finger protein 277",
  "gene_symbol": "ZNF277",
  "term_label": "Unknown biological process",
  "term_id": "UNKNOWN:0002"
}